{
  "gene_symbol": "SLC16A11",
  "term_label": "monocarboxylic acid transmembrane transporter activity",
  "gene_name": "Monocarboxylate transporter 11",
  "term_id": "GO:0008028",
  "gene": "UniProtKB:Q8NCK7"
}